alpha-1,6-mannosylglycoprotein 6-beta-N-acetylglucosaminyltransferase activity [GO:0030144] (molecular function) Relationships: is a type of acetylglucosaminyltransferase activity [GO:0008375]; is a type of GO:0140103 Also known as: alpha-1,3(6)-mannosylglycoprotein beta-1,6-N-acetylglucosaminyltransferase activity, alpha-1,6-mannosyl-glycoprotein 6-beta-N-acetylglucosaminyltransferase activity, GnTV activity, N-acetylglucosaminyltransferase V activity, UDP-N-acetyl-D-glucosamine:6-[2-(N-acetyl-beta-D-glucosaminyl)-alpha-D-mannosyl]-glycoprotein 6-beta-N-acetyl-D-glucosaminyltransferase activity, UDP-N-acetylglucosamine:alpha-mannoside-beta-1,6 N-acetylglucosaminyltransferase activity, UDP-N-acetylglucosamine:alpha-mannoside-beta1,6 N-acetylglucosaminyltransferase activity, alpha-mannoside beta-1,6-N-acetylglucosaminyltransferase activity, uridine diphosphoacetylglucosamine-alpha-mannoside beta-1->6-acetylglucosaminyltransferase activity, uridine diphosphoacetylglucosamine-alpha-mannoside beta1->6-acetylglucosaminyltransferase activity Sources: EC:2.4.1.155 Definition: Catalysis of the reaction: UDP-N-acetyl-D-glucosamine + N-acetyl-beta-D-glucosaminyl-1,2-alpha-D-mannosyl-1,3(6)-(N-acetyl-beta-D-glucosaminyl-1,2-alpha-D-mannosyl,1,6(3))-beta-D-mannosyl-1,4-N-acetyl-beta-D-glucosaminyl-R = UDP + N-acetyl-beta-D-glucosaminyl-1,2-(N-acetyl-beta-D-glucosaminyl-1,6)-1,2-alpha-D-mannosyl-1,3(6)-(N-acetyl-beta-D-glucosaminyl-1,2-alpha-D-mannosyl-1,6(3))-beta-D-mannosyl-1,4-N-acetyl-beta-D-glucosaminyl-R. Only branched mannose glycopeptides with non-reducing N-acetylglucosamine terminal residues act as acceptors.